{
  "gene_symbol": "PNCK",
  "gene_name": "Calcium_calmodulin-dependent protein kinase type 1B",
  "gene": "UniProtKB:Q6P2M8",
  "term_label": "cytoplasm",
  "term_id": "GO:0005737"
}